{
  "gene": "UniProtKB:P59537",
  "gene_name": "Taste receptor type 2 member 43",
  "term_id": "GO:0016020",
  "term_label": "membrane",
  "gene_symbol": "TAS2R43"
}